{
  "gene": "UniProtKB:Q13183",
  "term_id": "GO:0071422",
  "gene_name": "Solute carrier family 13 member 2",
  "gene_symbol": "SLC13A2",
  "term_label": "succinate transmembrane transport"
}